regulation of double-strand break repair via single-strand annealing, removal of nonhomologous ends [GO:1903776] (biological process) Definition: Any process that modulates the frequency, rate or extent of double-strand break repair via single-strand annealing, removal of nonhomologous ends. References: PMID:25203555 Sources: GOC:TermGenie, GO_REF:0000058 Relationships: is a type of regulation of double-strand break repair [GO:2000779]; regulates double-strand break repair via single-strand annealing, removal of nonhomologous ends [GO:0000736]